{
  "gene_symbol": "CHD3",
  "gene_name": "Chromodomain-helicase-DNA-binding protein 3",
  "term_label": "chromatin",
  "gene": "UniProtKB:Q12873",
  "term_id": "GO:0000785"
}